{
  "gene": "UniProtKB:Q8WXQ3",
  "term_id": "UNKNOWN:0001",
  "gene_name": "Putative uncharacterized protein encoded by LINC01599",
  "gene_symbol": "LINC01599",
  "term_label": "Unknown molecular function"
}